adenosylhomocysteinase activity [GO:0004013] (molecular function) Relationships: is_a hydrolase activity, acting on carbon-sulfur bonds [GO:0046508] Also known as: S-adenosylhomocysteine hydrolase activity, AdoHcyase activity, S-adenosyl-L-homocysteine hydrolase activity, S-adenosylhomocysteinase activity, S-adenosylhomocysteine synthase activity, SAHase activity, adenosylhomocysteine hydrolase activity Sources: RHEA:21708 Definition: Catalysis of the reaction: S-adenosyl-L-homocysteine + H2O = adenosine + L-homocysteine.